{
  "gene_name": "Tubulin gamma-1 chain",
  "gene_symbol": "TUBG1",
  "gene": "UniProtKB:P23258",
  "term_id": "GO:0007052",
  "term_label": "mitotic spindle organization"
}